{
  "gene_name": "Mitochondrial import inner membrane translocase subunit Tim10 B",
  "term_label": "protein transporter activity",
  "term_id": "GO:0140318",
  "gene": "UniProtKB:Q9Y5J6",
  "gene_symbol": "TIMM10B"
}